{
  "term_label": "S-adenosylmethionine cycle",
  "term_id": "GO:0033353",
  "gene_symbol": "AHCYL1",
  "gene": "UniProtKB:O43865",
  "gene_name": "S-adenosylhomocysteine hydrolase-like protein 1"
}